{
  "gene_symbol": "IGKV1-13",
  "gene": "UniProtKB:P0DP09",
  "term_id": "GO:0006955",
  "gene_name": "Immunoglobulin kappa variable 1-13",
  "term_label": "immune response"
}